cutinase activity [GO:0050525] (molecular function) Definition: Catalysis of the reaction: cutin + H2O = cutin monomers. Sources: EC:3.1.1.74, MetaCyc:3.1.1.74-RXN Also known as: cutin hydrolase activity Relationships: is a type of carboxylic ester hydrolase activity [GO:0052689]